{
  "gene": "UniProtKB:Q32NC0",
  "term_label": "Unknown molecular function",
  "gene_symbol": "C18orf21",
  "gene_name": "UPF0711 protein C18orf21",
  "term_id": "UNKNOWN:0001"
}